regulation of aldosterone metabolic process [GO:0032344] (biological process) Relationships: is a type of regulation of ketone metabolic process [GO:0010565]; is a type of regulation of steroid metabolic process [GO:0019218]; is a type of GO:0032350; is a type of GO:0062012; regulates aldosterone metabolic process [GO:0032341] Also known as: regulation of aldosterone metabolism Definition: Any process that modulates the frequency, rate or extent of the chemical reactions and pathways involving aldosterone. Subtypes: regulation of aldosterone biosynthetic process [GO:0032347] Sources: GOC:mah